{
  "term_id": "GO:0004340",
  "gene_symbol": "HKDC1",
  "gene_name": "Hexokinase HKDC1",
  "gene": "UniProtKB:Q2TB90",
  "term_label": "glucokinase activity"
}